{
  "gene_name": "Protein cornichon homolog 3",
  "gene": "UniProtKB:Q8TBE1",
  "term_id": "GO:0035249",
  "gene_symbol": "CNIH3",
  "term_label": "synaptic transmission, glutamatergic"
}